{
  "gene_symbol": "SLC6A13",
  "gene_name": "Sodium- and chloride-dependent GABA transporter 2",
  "term_id": "GO:0035725",
  "gene": "UniProtKB:Q9NSD5",
  "term_label": "sodium ion transmembrane transport"
}